{
  "gene_symbol": "VAMP1",
  "gene": "UniProtKB:P23763",
  "gene_name": "Vesicle-associated membrane protein 1",
  "term_label": "syntaxin binding",
  "term_id": "GO:0019905"
}